{
  "gene_name": "Schlafen family member 11",
  "term_label": "tRNA binding",
  "gene_symbol": "SLFN11",
  "gene": "UniProtKB:Q7Z7L1",
  "term_id": "GO:0000049"
}